glyceraldehyde-3-phosphate biosynthetic process [GO:0046166] (biological process) Definition: The chemical reactions and pathways resulting in the formation of glyceraldehyde-3-phosphate, an important intermediate in glycolysis. Relationships: is a type of glyceraldehyde-3-phosphate metabolic process [GO:0019682]; is a type of aldehyde biosynthetic process [GO:0046184]; is a type of organophosphate biosynthetic process [GO:0090407]; is a type of carbohydrate derivative biosynthetic process [GO:1901137] Also known as: glyceraldehyde 3-phosphate biosynthesis, glyceraldehyde 3-phosphate biosynthetic process, glyceraldehyde-3-phosphate anabolism, glyceraldehyde-3-phosphate biosynthesis, glyceraldehyde-3-phosphate formation, glyceraldehyde-3-phosphate synthesis Sources: GOC:ai